ectoderm development [GO:0007398] (biological process) Definition: The process whose specific outcome is the progression of the ectoderm over time, from its formation to the mature structure. In animal embryos, the ectoderm is the outer germ layer of the embryo, formed during gastrulation. Sources: GOC:dph, GOC:tb Regulation: RO_0002211 by GO:2000383; negatively regulated by GO:2000384; positively regulated by GO:2000385 Relationships: is a type of tissue development [GO:0009888]